IDP catabolic process [GO:0046709] (biological process) Relationships: is a type of purine ribonucleotide catabolic process [GO:0009154]; is a type of GO:0009181; is a type of IDP metabolic process [GO:0046707] Sources: GOC:ai Also known as: IDP breakdown, IDP catabolism, IDP degradation Definition: The chemical reactions and pathways resulting in the breakdown of IDP, inosine 5'-diphosphate.